{
  "gene_name": "Protein max",
  "term_id": "GO:0003700",
  "gene_symbol": "MAX",
  "term_label": "DNA-binding transcription factor activity",
  "gene": "UniProtKB:P61244"
}